L-ribulose-phosphate 4-epimerase activity [GO:0008742] (molecular function) Relationships: is a type of GO:0016857 Also known as: L-ribulose-5-phosphate 4-epimerase, AraD, L-Ru5P, L-ribulose 5-phosphate 4-epimerase activity, L-ru5P activity, phosphoribulose isomerase activity, ribulose phosphate 4-epimerase activity Definition: Catalysis of the reaction: L-ribulose 5-phosphate = D-xylulose 5-phosphate. Sources: EC:5.1.3.4, RHEA:22368